negative regulation of aggregate size involved in sorocarp development [GO:0031158] (biological process) Relationships: is a type of regulation of aggregate size involved in sorocarp development [GO:0031157] Also known as: down regulation of aggregate size, down-regulation of aggregate size, downregulation of aggregate size, inhibition of aggregate size Definition: Any process that decreases the size of the aggregate formed during sorocarp formation. References: PMID:5002049 Sources: GOC:mah, GOC:mtg_sensu, GOC:pg